extrinsic component of postsynaptic early endosome membrane [GO:0098998] (cellular component) Relationships: is a type of extrinsic component of postsynaptic endosome membrane [GO:0098999]; is part of GO:0098896 Definition: The component of the postsynaptic early endosome membrane consisting of gene products and protein complexes that are loosely bound to one of its surfaces, but not integrated into the hydrophobic region. Sources: GOC:autophagy, GOC:mf